{
  "term_label": "Unknown molecular function",
  "gene_symbol": "ENHO",
  "gene_name": "Adropin",
  "term_id": "UNKNOWN:0001",
  "gene": "UniProtKB:Q6UWT2"
}